xylan 1,3-beta-xylosidase activity [GO:0033914] (molecular function) Definition: Catalysis of the hydrolysis of successive xylose residues from the non-reducing termini of (1->3)-beta-D-xylans. Sources: EC:3.2.1.72 Also known as: 1,3-beta-D-xylan xylohydrolase activity, 1,3-beta-D-xylosidase, exo-1,3-beta-xylosidase activity, beta-1,3'-xylanase activity, exo-1,3-beta-xylosidase activity, exo-beta-1,3'-xylanase activity Relationships: is a type of xylanase activity [GO:0097599]